{
  "term_id": "GO:0019827",
  "gene_name": "Brain-specific homeobox protein homolog",
  "gene_symbol": "BSX",
  "term_label": "stem cell population maintenance",
  "gene": "UniProtKB:Q3C1V8"
}